{
  "gene_name": "Immunoglobulin kappa variable 1-13",
  "gene": "UniProtKB:P0DP09",
  "term_label": "immunoglobulin complex",
  "term_id": "GO:0019814",
  "gene_symbol": "IGKV1-13"
}